B cell costimulation [GO:0031296] (BP) Definition: The process of providing, via surface-bound receptor-ligand pairs, a second, antigen-independent, signal in addition to that provided by the B cell receptor to augment B cell activation. Sources: ISBN:0781735149 Also known as: B cell co-stimulation, B lymphocyte co-stimulation, B lymphocyte costimulation, B-cell co-stimulation, B-cell costimulation, B-lymphocyte co-stimulation, B-lymphocyte costimulation Relationships: is a type of GO:0031294; is a type of positive regulation of B cell activation [GO:0050871]